{
  "gene_symbol": "SCNN1D",
  "gene_name": "Amiloride-sensitive sodium channel subunit delta",
  "term_id": "GO:0015280",
  "term_label": "ligand-gated sodium channel activity",
  "gene": "UniProtKB:P51172"
}